{
  "term_label": "forebrain neuron development",
  "gene": "UniProtKB:Q68G74",
  "term_id": "GO:0021884",
  "gene_name": "LIM_homeobox protein Lhx8",
  "gene_symbol": "LHX8"
}